arachidonate metabolite production involved in inflammatory response [GO:0002538] (biological process) Definition: The synthesis or release of products of arachidonic acid metabolism following a stimulus as part of an inflammatory response, resulting in an increase in their intracellular or extracellular levels. Also known as: arachidonic acid metabolite production involved in acute inflammatory response, production of arachidonic acid metabolites involved in acute inflammatory response, arachidonic acid metabolite production involved in inflammatory response, production of arachidonic acid metabolites involved in inflammatory response Sources: GOC:add, ISBN:0781735149 Subtypes: prostaglandin production involved in inflammatory response [GO:0002539], GO:0002540 Relationships: is a type of production of molecular mediator involved in inflammatory response [GO:0002532]